cellular response to phenylpropanoid [GO:1905546] (biological process) Subtypes: cellular response to hydroxyisoflavone [GO:0071413], GO:1902169 References: PMID:22700048 Sources: GOC:TermGenie, GO_REF:0000071 Definition: Any process that results in a change in state or activity of a cell (in terms of movement, secretion, enzyme production, gene expression, etc.) as a result of a phenylpropanoid stimulus. Relationships: is a type of cellular response to chemical stimulus [GO:0070887]; is a type of GO:0080184